{
  "gene": "UniProtKB:Q8NGH6",
  "gene_symbol": "OR52L2P",
  "gene_name": "Putative olfactory receptor 52L2",
  "term_id": "GO:0004984",
  "term_label": "olfactory receptor activity"
}